{
  "gene": "UniProtKB:P33778",
  "gene_symbol": "H2BC3",
  "term_label": "DNA binding",
  "gene_name": "Histone H2B type 1-B",
  "term_id": "GO:0003677"
}